{
  "term_label": "regulation of macrophage activation",
  "gene_symbol": "SHPK",
  "gene": "UniProtKB:Q9UHJ6",
  "gene_name": "Sedoheptulokinase",
  "term_id": "GO:0043030"
}